{
  "gene_name": "Transmembrane emp24 domain-containing protein 3",
  "term_label": "COPII-coated ER to Golgi transport vesicle",
  "term_id": "GO:0030134",
  "gene_symbol": "TMED3",
  "gene": "UniProtKB:Q9Y3Q3"
}